negative regulation of glycogen metabolic process [GO:0070874] (biological process) Definition: Any process that stops, prevents, or reduces the frequency, rate or extent of the chemical reactions and pathways involving glycogen. Sources: GOC:mah Also known as: negative regulation of glycogen metabolism Relationships: is a type of negative regulation of macromolecule metabolic process [GO:0010605]; is_a negative regulation of carbohydrate metabolic process [GO:0045912]; is a type of regulation of glycogen metabolic process [GO:0070873]; negatively regulates glycogen metabolic process [GO:0005977] Subtypes: negative regulation of glycogen biosynthetic process [GO:0045719], negative regulation of glycogen catabolic process [GO:0045818]